lncRNA catabolic process [GO:0110064] (biological process) Subtypes: GO:0180036 Relationships: is a type of GO:0006401 References: PMID:24493644 Sources: GOC:al Definition: The chemical reactions and pathways resulting in the breakdown of lncRNAs, non-coding RNAs over 200 nucleotides in length. Also known as: lncRNA breakdown, lncRNA catabolism, lncRNA degradation